{
  "gene_symbol": "TBC1D15",
  "term_id": "UNKNOWN:0003",
  "term_label": "Unknown cellular component",
  "gene": "UniProtKB:Q8TC07",
  "gene_name": "TBC1 domain family member 15"
}